{
  "gene": "UniProtKB:Q9UP65",
  "gene_name": "Cytosolic phospholipase A2 gamma",
  "term_label": "glycerophospholipid catabolic process",
  "term_id": "GO:0046475",
  "gene_symbol": "PLA2G4C"
}